{
  "gene_symbol": "IL36B",
  "gene": "UniProtKB:Q9NZH7",
  "term_label": "cytokine-mediated signaling pathway",
  "term_id": "GO:0019221",
  "gene_name": "Interleukin-36 beta"
}